{
  "term_label": "sarcoplasmic reticulum",
  "gene": "UniProtKB:Q8NF91",
  "gene_symbol": "SYNE1",
  "gene_name": "Nesprin-1",
  "term_id": "GO:0016529"
}